positive regulation of fat cell apoptotic process [GO:1904651] (biological process) Relationships: is a type of GO:0043065; is a type of regulation of fat cell apoptotic process [GO:1904649]; positively regulates fat cell apoptotic process [GO:1904606] Also known as: positive regulation of adipocyte apoptotic process, positive regulation of adipose cell apoptotic process, up regulation of adipocyte apoptotic process, up regulation of adipose cell apoptotic process, up regulation of fat cell apoptotic process, up-regulation of adipocyte apoptotic process, up-regulation of adipose cell apoptotic process, up-regulation of fat cell apoptotic process, upregulation of adipocyte apoptotic process, upregulation of adipose cell apoptotic process, upregulation of fat cell apoptotic process, activation of adipocyte apoptosis, activation of adipocyte apoptotic process, activation of adipose cell apoptosis, activation of adipose cell apoptotic process, activation of fat cell apoptosis, activation of fat cell apoptotic process, positive regulation of adipocyte apoptosis, positive regulation of adipose cell apoptosis, positive regulation of fat cell apoptosis, up regulation of adipocyte apoptosis, up regulation of adipose cell apoptosis, up regulation of fat cell apoptosis, up-regulation of adipocyte apoptosis, up-regulation of adipose cell apoptosis, up-regulation of fat cell apoptosis, upregulation of adipocyte apoptosis, upregulation of adipose cell apoptosis, upregulation of fat cell apoptosis References: PMID:17024416 Sources: GOC:TermGenie, GO_REF:0000058 Definition: Any process that activates or increases the frequency, rate or extent of fat cell apoptotic process.